positive regulation of ureter smooth muscle cell differentiation [GO:2000063] (biological process) Sources: GOC:mtg_kidney_jan10, GOC:obol, GOC:yaf Relationships: is a type of GO:0051152; is a type of positive regulation of multicellular organismal process [GO:0051240]; is a type of regulation of ureter smooth muscle cell differentiation [GO:2000061]; positively regulates ureter smooth muscle cell differentiation [GO:0072193] Definition: Any process that activates or increases the frequency, rate or extent of ureter smooth muscle cell differentiation.